{
  "gene_symbol": "HLF",
  "gene_name": "Hepatic leukemia factor",
  "term_id": "GO:0000978",
  "gene": "UniProtKB:Q16534",
  "term_label": "RNA polymerase II cis-regulatory region sequence-specific DNA binding"
}